oligopeptide export from mitochondrion [GO:0090374] (biological process) Definition: The process in which an oligopeptide is transported out of the mitochondrial matrix. Oligopeptides are molecules that contain a small number (2 to 20) of amino-acid residues connected by peptide linkages. References: PMID:11251115 Relationships: is a type of oligopeptide transmembrane transport [GO:0035672]